{
  "gene_symbol": "RPP25",
  "term_id": "GO:0001682",
  "gene_name": "Ribonuclease P protein subunit p25",
  "gene": "UniProtKB:Q9BUL9",
  "term_label": "tRNA 5'-leader removal"
}